{
  "term_label": "DNA binding",
  "term_id": "GO:0003677",
  "gene": "UniProtKB:Q9UBC3",
  "gene_symbol": "DNMT3B",
  "gene_name": "DNA (cytosine-5)-methyltransferase 3B"
}